{
  "term_id": "GO:0046854",
  "gene": "UniProtKB:O14986",
  "term_label": "phosphatidylinositol phosphate biosynthetic process",
  "gene_name": "Phosphatidylinositol 4-phosphate 5-kinase type-1 beta",
  "gene_symbol": "PIP5K1B"
}